{
  "gene": "UniProtKB:P55209",
  "gene_name": "Nucleosome assembly protein 1-like 1",
  "term_label": "nucleosome assembly",
  "term_id": "GO:0006334",
  "gene_symbol": "NAP1L1"
}